{
  "term_id": "GO:0005125",
  "gene_name": "Protein Wnt-6",
  "gene": "UniProtKB:Q9Y6F9",
  "gene_symbol": "WNT6",
  "term_label": "cytokine activity"
}